{
  "gene_symbol": "SET",
  "gene": "UniProtKB:Q01105",
  "term_id": "GO:0000785",
  "term_label": "chromatin",
  "gene_name": "Protein SET"
}